{
  "gene": "UniProtKB:O15554",
  "term_id": "GO:0043005",
  "term_label": "neuron projection",
  "gene_symbol": "KCNN4",
  "gene_name": "Intermediate conductance calcium-activated potassium channel protein 4"
}